{
  "term_id": "GO:0099550",
  "gene_name": "Cerebellin-3",
  "gene": "UniProtKB:Q6UW01",
  "gene_symbol": "CBLN3",
  "term_label": "trans-synaptic signaling, modulating synaptic transmission"
}